{
  "gene_name": "Interleukin-34",
  "gene": "UniProtKB:Q6ZMJ4",
  "gene_symbol": "IL34",
  "term_id": "GO:0005157",
  "term_label": "macrophage colony-stimulating factor receptor binding"
}